{
  "gene": "UniProtKB:A0A0B4J271",
  "term_label": "peptide antigen binding",
  "gene_name": "T cell receptor alpha variable 12-3",
  "term_id": "GO:0042605",
  "gene_symbol": "TRAV12-3"
}